{
  "term_id": "UNKNOWN:0002",
  "gene_symbol": "IGFLR1",
  "gene": "UniProtKB:Q9H665",
  "gene_name": "IGF-like family receptor 1",
  "term_label": "Unknown biological process"
}